mesoderm formation [GO:0001707] (biological process) Subtypes: axial mesoderm formation [GO:0048320], GO:0048341, GO:0048370, intermediate mesoderm formation [GO:0048391] Relationships: is a type of formation of primary germ layer [GO:0001704]; is part of mesoderm morphogenesis [GO:0048332] Definition: The process that gives rise to the mesoderm. This process pertains to the initial formation of the structure from unspecified parts. Regulation: regulated by regulation of mesoderm formation [GO:1905902]; negatively regulated by negative regulation of mesoderm formation [GO:1905903]; positively regulated by positive regulation of mesoderm formation [GO:1905904] Sources: GOC:go_curators